{
  "term_label": "Unknown molecular function",
  "gene": "UniProtKB:Q96J86",
  "term_id": "UNKNOWN:0001",
  "gene_symbol": "CYYR1",
  "gene_name": "Cysteine and tyrosine-rich protein 1"
}